negative regulation of mesenchymal cell apoptotic process involved in nephron morphogenesis [GO:0072040] (biological process) Definition: Any process that reduces the occurrence or rate of mesenchymal stem cell death by apoptotic process that contributes to the shaping of the nephron. Sources: GOC:mtg_apoptosis, GOC:mtg_kidney_jan10 Subtypes: GO:0061296, negative regulation of mesenchymal cell apoptotic process involved in metanephric nephron morphogenesis [GO:0072305] Relationships: is a type of regulation of mesenchymal cell apoptotic process involved in nephron morphogenesis [GO:0072039]; is a type of negative regulation of apoptotic process involved in morphogenesis [GO:1902338]; is a type of negative regulation of somatic stem cell population maintenance [GO:1904673]; is a type of negative regulation of mesenchymal cell apoptotic process [GO:2001054]; negatively regulates mesenchymal stem cell maintenance involved in nephron morphogenesis [GO:0072038]; negatively regulates mesenchymal cell apoptotic process involved in nephron morphogenesis [GO:1901145] Also known as: negative regulation of mesenchymal stem cell apoptotic process involved in nephron morphogenesis, negative regulation of mesenchymal stem cell apoptosis involved in nephron morphogenesis